nuclear cell cycle DNA replication initiation [GO:1902315] (biological process) Relationships: is a type of cell cycle DNA replication initiation [GO:1902292]; is part of GO:0033260 Sources: GOC:TermGenie, GOC:mtg_cell_cycle Definition: Any DNA replication initiation that is involved in nuclear cell cycle DNA replication. Subtypes: GO:1902974, GO:1902975 Also known as: DNA replication initiation involved in nuclear cell cycle DNA replication, DNA endoreduplication initiation involved in nuclear cell cycle DNA replication, DNA re-replication initiation involved in nuclear cell cycle DNA replication